non-phosphorylated glucose catabolic process [GO:0019595] (biological process) Subtypes: Entner-Doudoroff pathway through gluconate to D-glyceraldehyde [GO:0061680] Definition: The chemical reactions and pathways resulting in the breakdown of non-phosphorylated forms of glucose. Relationships: is a type of glucose catabolic process [GO:0006007] Sources: GOC:ai Also known as: non-phosphorylated glucose breakdown, non-phosphorylated glucose catabolism, non-phosphorylated glucose degradation